{
  "term_id": "GO:0000981",
  "gene": "UniProtKB:P0CH99",
  "gene_name": "Zinc finger protein 705D",
  "gene_symbol": "ZNF705D",
  "term_label": "DNA-binding transcription factor activity, RNA polymerase II-specific"
}